cell migration involved in coronary vasculogenesis [GO:0060980] (biological process) Sources: GOC:mtg_heart Definition: The orderly movement of a cell from one site to another that will contribute to the differentiation of an endothelial cell that will form the blood vessels of the heart. Relationships: is a type of GO:0035441; is_a GO:0060973; is part of vasculogenesis involved in coronary vascular morphogenesis [GO:0060979]